behavioral defense response to insect [GO:0002211] (biological process) Sources: GOC:add Definition: A behavioral response seeking to protect an organism from an a perceived external threat from an insect or insects to that organism. Also known as: behavioural defense response to insect Relationships: is a type of GO:0002209; is a type of defense response to insect [GO:0002213]